{
  "gene_symbol": "SPATA19",
  "term_id": "UNKNOWN:0001",
  "term_label": "Unknown molecular function",
  "gene": "UniProtKB:Q7Z5L4",
  "gene_name": "Spermatogenesis-associated protein 19, mitochondrial"
}